{
  "term_label": "Unknown cellular component",
  "gene_name": "Protein FAM24B",
  "gene": "UniProtKB:Q8N5W8",
  "term_id": "UNKNOWN:0003",
  "gene_symbol": "FAM24B"
}